{
  "gene": "UniProtKB:Q8ND90",
  "term_id": "UNKNOWN:0003",
  "gene_name": "Paraneoplastic antigen Ma1",
  "gene_symbol": "PNMA1",
  "term_label": "Unknown cellular component"
}